synaptic assembly at neuromuscular junction [GO:0051124] (biological process) References: PMID:20215342 Relationships: is a type of synapse assembly [GO:0007416]; is a type of neuromuscular junction development [GO:0007528]; is a type of GO:0048589 Also known as: cholinergic synaptogenesis, synaptic growth at neuromuscular junction Regulation: regulated by regulation of synaptic assembly at neuromuscular junction [GO:0008582]; negatively regulated by negative regulation of synaptic assembly at neuromuscular junction [GO:0045886]; positively regulated by positive regulation of synaptic assembly at neuromuscular junction [GO:0045887] Definition: The assembly of a synapse at a neuromuscular junction.